{
  "gene": "UniProtKB:P62312",
  "term_id": "GO:0003723",
  "gene_name": "U6 snRNA-associated Sm-like protein LSm6",
  "gene_symbol": "LSM6",
  "term_label": "RNA binding"
}